{
  "term_label": "A band",
  "term_id": "GO:0031672",
  "gene": "UniProtKB:Q2TBA0",
  "gene_symbol": "KLHL40",
  "gene_name": "Kelch-like protein 40"
}